thebaine 6-O-demethylase activity [GO:0102802] (molecular function) Definition: Catalysis of the reaction: thebaine + 2-oxoglutarate + O2 = neopinone + formaldehyde + succinate + carbon dioxide. Sources: EC:1.14.11.31, GOC:pz Relationships: is a type of 2-oxoglutarate-dependent dioxygenase activity [GO:0016706]